5-hydroxymethyluracil DNA N-glycosylase activity [GO:0034043] (molecular function) Relationships: is a type of oxidized pyrimidine nucleobase lesion DNA N-glycosylase activity [GO:0000703] Definition: Catalysis of the removal of 5-hydroxymethyluracil bases by cleaving the N-C1' glycosidic bond between the oxidized pyrimidine and the deoxyribose sugar. References: PMID:17641464 Sources: GOC:mah Also known as: 5-hmU DNA N-glycosylase activity